{
  "term_label": "ornithine decarboxylase inhibitor activity",
  "gene_name": "Ornithine decarboxylase antizyme 2",
  "gene": "UniProtKB:O95190",
  "term_id": "GO:0008073",
  "gene_symbol": "OAZ2"
}